{
  "gene_name": "Carbonic anhydrase-related protein 11",
  "term_label": "hydro-lyase activity",
  "term_id": "GO:0016836",
  "gene_symbol": "CA11",
  "gene": "UniProtKB:O75493"
}